neuromast hair cell development [GO:0035675] (BP) Sources: CL:0000856 Subtypes: GO:0035676, GO:0035677 Definition: The process whose specific outcome is the progression of a neuromast hair cell over time, from its formation to the mature structure. A neuromast hair cell is a hair cell that acts as a sensory receptor of the neuromast; it is morphologically polarized as a result of the relative position of the single kinocilium and the clusters of stereocilia on its apical surface. Cell development does not include the steps involved in committing a cell to a specific fate. Relationships: is a type of neuron development [GO:0048666]; is part of GO:0048886